{
  "gene_symbol": "DNAJC7",
  "gene": "UniProtKB:Q99615",
  "term_label": "Unknown biological process",
  "gene_name": "DnaJ homolog subfamily C member 7",
  "term_id": "UNKNOWN:0002"
}